{
  "gene_symbol": "PARVB",
  "gene_name": "Beta-parvin",
  "term_label": "actin binding",
  "gene": "UniProtKB:Q9HBI1",
  "term_id": "GO:0003779"
}